{
  "gene_symbol": "GBF1",
  "term_id": "GO:0000137",
  "gene": "UniProtKB:Q92538",
  "term_label": "Golgi cis cisterna",
  "gene_name": "Golgi-specific brefeldin A-resistance guanine nucleotide exchange factor 1"
}